glutamate binding [GO:0016595] (molecular function) Definition: Binding to glutamate, the anion of 2-aminopentanedioic acid. Sources: GOC:ai Relationships: is_a GO:0016597; is a type of GO:0031406 Also known as: glutamic acid binding